{
  "gene_name": "NADH dehydrogenase [ubiquinone] flavoprotein 3, mitochondrial",
  "gene_symbol": "NDUFV3",
  "term_id": "UNKNOWN:0001",
  "term_label": "Unknown molecular function",
  "gene": "UniProtKB:P56181"
}